multivesicular body, internal vesicle lumen [GO:0097489] (cellular component) References: PMID:21183070 Sources: GOC:pde Definition: The volume enclosed by the membrane of the multivesicular body internal vesicle. Relationships: is a type of GO:0031983; is a type of intracellular organelle lumen [GO:0070013]; is part of GO:0097487